{
  "gene_name": "Translation initiation factor eIF-2B subunit gamma",
  "gene_symbol": "EIF2B3",
  "term_id": "GO:0005085",
  "gene": "UniProtKB:Q9NR50",
  "term_label": "guanyl-nucleotide exchange factor activity"
}